leading edge cell differentiation [GO:0035026] (biological process) Definition: The process in which relatively unspecialized cells acquire specialized structural and/or functional features of leading edge cells, cells at the front of a migrating epithelial sheet. Subtypes: dorsal closure, leading edge cell differentiation [GO:0046663] Sources: GOC:bf Relationships: is a type of epithelial cell differentiation [GO:0030855]